{
  "term_id": "GO:0006508",
  "gene_name": "A disintegrin and metalloproteinase with thrombospondin motifs 15",
  "gene": "UniProtKB:Q8TE58",
  "gene_symbol": "ADAMTS15",
  "term_label": "proteolysis"
}